{
  "gene_symbol": "KHDC3L",
  "gene_name": "KH domain-containing protein 3",
  "term_id": "UNKNOWN:0002",
  "term_label": "Unknown biological process",
  "gene": "UniProtKB:Q587J8"
}